prostate induction [GO:0060514] (biological process) References: PMID:18977204 Sources: GOC:dph Relationships: is a type of organ induction [GO:0001759]; is_a GO:0060685; is a type of positive regulation of morphogenesis of an epithelium [GO:1905332]; is a type of positive regulation of reproductive process [GO:2000243]; positively regulates prostate field specification [GO:0060515] Definition: The close range interaction of the urogenital sinus mesenchyme and the urogenital sinus epithelium that causes the cells of the urogenital sinus epithelium to change their fates and specify the development of the prostate gland.